{
  "term_id": "GO:0005615",
  "term_label": "extracellular space",
  "gene_symbol": "IHH",
  "gene_name": "Indian hedgehog protein",
  "gene": "UniProtKB:Q14623"
}